{
  "gene": "UniProtKB:Q86TZ1",
  "term_label": "Unknown biological process",
  "gene_name": "Tetratricopeptide repeat protein 6",
  "gene_symbol": "TTC6",
  "term_id": "UNKNOWN:0002"
}